{
  "gene": "UniProtKB:Q8WWV3",
  "term_label": "alcohol dehydrogenase [NAD(P)+] activity",
  "term_id": "GO:0018455",
  "gene_name": "Reticulon-4-interacting protein 1, mitochondrial",
  "gene_symbol": "RTN4IP1"
}